{
  "gene_name": "Guanine nucleotide-binding protein G(t) subunit alpha-3",
  "gene": "UniProtKB:A8MTJ3",
  "term_id": "GO:0001664",
  "term_label": "G protein-coupled receptor binding",
  "gene_symbol": "GNAT3"
}